somitogenesis [GO:0001756] (biological process) Relationships: is a type of GO:0009952; is a type of segmentation [GO:0035282]; is a type of anatomical structure formation involved in morphogenesis [GO:0048646]; is part of GO:0043009; is part of somite development [GO:0061053] Sources: ISBN:0721662544 Also known as: formation of mesodermal clusters Definition: The formation of mesodermal clusters that are arranged segmentally along the anterior posterior axis of an embryo. Regulation: regulated by regulation of somitogenesis [GO:0014807]